sphingomyelin catabolic process [GO:0006685] (biological process) Sources: ISBN:0198506732 Also known as: sphingomyelin breakdown, sphingomyelin catabolism, sphingomyelin degradation Definition: The chemical reactions and pathways resulting in the breakdown of sphingomyelin, N-acyl-4-sphingenyl-1-O-phosphorylcholine. Regulation: regulated by regulation of sphingomyelin catabolic process [GO:2000754]; positively regulated by positive regulation of sphingomyelin catabolic process [GO:2000755] Relationships: is a type of sphingomyelin metabolic process [GO:0006684]; is a type of GO:0009395; is a type of sphingolipid catabolic process [GO:0030149]